{
  "term_id": "GO:0031431",
  "gene_symbol": "DBF4B",
  "gene_name": "Protein DBF4 homolog B",
  "gene": "UniProtKB:Q8NFT6",
  "term_label": "Dbf4-dependent protein kinase complex"
}